{
  "term_id": "GO:1990573",
  "gene_symbol": "SLC12A1",
  "gene_name": "Solute carrier family 12 member 1",
  "gene": "UniProtKB:Q13621",
  "term_label": "potassium ion import across plasma membrane"
}